{
  "term_label": "RNA binding",
  "gene_symbol": "HNRNPCL4",
  "gene_name": "Heterogeneous nuclear ribonucleoprotein C-like 4",
  "gene": "UniProtKB:P0DMR1",
  "term_id": "GO:0003723"
}